ubiquitin-modified protein reader activity [GO:0140036] (molecular function) Relationships: is a type of ubiquitin-like protein reader activity [GO:0140035] Subtypes: ubiquitin-modified histone reader activity [GO:0061649] Definition: A molecular adaptor recognizes and binds a target protein containing a ubiquitination modification and brings the target protein into contact with another protein to allow those proteins to function in a coordinated way. Also known as: ubiquitin-dependent protein binding References: PMID:26060076 Note: This term should only be used when the binding is shown to require ubiquitination of the target protein: the interaction needs to be tested with and without the PTM. The binding does not need to be at the site of ubiquitination. It may be that the ubiquitination causes a conformational change that allows binding of the protein to another region; this type of ubiquitination-dependent protein binding is valid for annotation to this term.